{
  "gene_symbol": "LETMD1",
  "term_label": "mitochondrion",
  "gene": "UniProtKB:Q6P1Q0",
  "gene_name": "LETM1 domain-containing protein 1",
  "term_id": "GO:0005739"
}